{
  "gene_name": "Follicle-stimulating hormone receptor",
  "gene_symbol": "FSHR",
  "term_label": "G protein-coupled peptide receptor activity",
  "term_id": "GO:0008528",
  "gene": "UniProtKB:P23945"
}